cell-matrix adhesion involved in tangential migration using cell-cell interactions [GO:0021833] (biological process) Definition: The interaction of a cell and the extracellular matrix involved in the directed tangential movement of cells mediated by cell-cell interactions in the developing cerebral cortex. Relationships: is a type of cell-substrate adhesion [GO:0031589]; is part of cerebral cortex tangential migration using cell-cell interactions [GO:0021823] References: PMID:12626695 Sources: GOC:ascb_2009, GOC:cls, GOC:dgh, GOC:dph, GOC:jid